{
  "gene_symbol": "SEPTIN8",
  "term_label": "cytoskeleton-dependent cytokinesis",
  "gene": "UniProtKB:Q92599",
  "gene_name": "Septin-8",
  "term_id": "GO:0061640"
}